{
  "term_label": "Unknown molecular function",
  "gene": "UniProtKB:Q9UKI3",
  "gene_symbol": "VPREB3",
  "gene_name": "Pre-B lymphocyte protein 3",
  "term_id": "UNKNOWN:0001"
}